{
  "gene_symbol": "NEDD8",
  "term_id": "GO:0030162",
  "term_label": "regulation of proteolysis",
  "gene": "UniProtKB:Q15843",
  "gene_name": "NEDD8"
}